regulation of rRNA stability [GO:0044357] (biological process) Definition: Any process that modulates the propensity of rRNA molecules to degradation. Includes processes that both stabilize and destabilize rRNAs. Sources: GOC:jl Also known as: regulation of ribosomal RNA stability Relationships: is a type of regulation of RNA stability [GO:0043487]; is a type of regulation of rRNA catabolic process [GO:1902374] Subtypes: GO:0044529